glial cell activation [GO:0061900] (biological process) Relationships: is a type of cell activation [GO:0001775]; is part of GO:0150076 References: PMID:18723082 Sources: GOC:aruk, GOC:bc Subtypes: microglial cell activation [GO:0001774], GO:0048143 Definition: A change in morphology and behavior of a glial cell resulting from exposure to a cytokine, chemokine, cellular ligand, or soluble factor.